{
  "term_id": "GO:0070032",
  "gene_name": "Synaptosomal-associated protein 25",
  "gene": "UniProtKB:P60880",
  "term_label": "synaptobrevin 2-SNAP-25-syntaxin-1a-complexin I complex",
  "gene_symbol": "SNAP25"
}